{
  "term_id": "GO:0050680",
  "gene_name": "Cyclin-dependent kinase inhibitor 1C",
  "term_label": "negative regulation of epithelial cell proliferation",
  "gene_symbol": "CDKN1C",
  "gene": "UniProtKB:P49918"
}